epicardium-derived cardiac fibroblast cell fate commitment [GO:0060941] (biological process) Relationships: is a type of cardiac fibroblast cell fate commitment [GO:0060937]; is part of GO:0060938 Sources: GOC:mtg_heart Definition: The commitment of an epicardial cell to a cardiac fibroblast cell fate and its capacity to differentiate into a cardiac fibroblast. A cardiac fibroblast is a connective tissue cell in the heart which secretes an extracellular matrix rich in collagen and other macromolecules.